2,3-dihydroxy-2,3-dihydro-p-cumate dehydrogenase activity [GO:0018511] (molecular function) Definition: Catalysis of the reaction: cis-2,3-dihydroxy-2,3-dihydro-p-cumate + NAD+ = 2,3-dihydroxy-p-cumate + H+ + NADH. Also known as: cis-2,3-dihydroxy-2,3-dihydro-p-cumate:NAD+ oxidoreductase activity Sources: EC:1.3.1.58, RHEA:23772 Relationships: is a type of GO:0016628